{
  "term_id": "GO:0009968",
  "gene": "UniProtKB:Q8TF42",
  "gene_name": "Ubiquitin-associated and SH3 domain-containing protein B",
  "gene_symbol": "UBASH3B",
  "term_label": "negative regulation of signal transduction"
}